maternal determination of dorsal/ventral axis, ovarian follicular epithelium, soma encoded [GO:0008071] (biological process) Relationships: is a type of dorsal/ventral axis specification, ovarian follicular epithelium [GO:0008069] Sources: GOC:mtg_sensu, ISBN:0879694238 Definition: Polarization of the ovarian follicle cells along the dorsal-ventral axis by a gene product encoded by somatic cells. An example of this process is found in Drosophila melanogaster. Also known as: maternal determination of dorsal/ventral axis, follicular epithelium, soma encoded, maternal determination of dorsal-ventral axis, ovarian follicular epithelium, soma encoded, maternal determination of dorsoventral axis, ovarian follicular epithelium, soma encoded